{
  "term_label": "guanyl-nucleotide exchange factor activity",
  "gene_name": "Translation initiation factor eIF-2B subunit alpha",
  "term_id": "GO:0005085",
  "gene_symbol": "EIF2B1",
  "gene": "UniProtKB:Q14232"
}